2-methoxy-6-polyprenolphenol 4-hydroxylase activity [GO:0120538] (MF) Definition: Catalysis of the reaction: 2-methoxy-6-(all-trans-polyprenyl)phenol + 2 reduced [2Fe-2S]-[ferredoxin] + O2 + 2 H+ = 2-methoxy-6-(all-trans-polyprenyl)benzene-1,4-diol + 2 oxidized [2Fe-2S]-[ferredoxin] + H2O. Relationships: is a type of oxidoreductase activity, acting on paired donors, with incorporation or reduction of molecular oxygen, reduced iron-sulfur protein as one donor, and incorporation of one atom of oxygen [GO:0016713]; BFO_0000050 GO:0006744 References: PMID:38425362 Sources: RHEA:81183